{
  "gene": "UniProtKB:Q9UKB1",
  "term_id": "GO:0043005",
  "term_label": "neuron projection",
  "gene_name": "F-box_WD repeat-containing protein 11",
  "gene_symbol": "FBXW11"
}